negative regulation of interleukin-1 production [GO:0032692] (BP) Also known as: down regulation of interleukin-1 production, down-regulation of interleukin-1 production, downregulation of interleukin-1 production, negative regulation of IL-1 production, inhibition of interleukin-1 production, negative regulation of interleukin-1 biosynthetic process, negative regulation of interleukin-1 secretion Sources: GOC:mah Relationships: is a type of negative regulation of cytokine production [GO:0001818]; is a type of GO:0032652; negatively regulates interleukin-1 production [GO:0032612] Subtypes: negative regulation of interleukin-1 alpha production [GO:0032690], negative regulation of interleukin-1 beta production [GO:0032691] Definition: Any process that stops, prevents, or reduces the frequency, rate, or extent of interleukin-1 production.